{
  "term_label": "DNA damage response",
  "term_id": "GO:0006974",
  "gene": "UniProtKB:P38936",
  "gene_name": "Cyclin-dependent kinase inhibitor 1",
  "gene_symbol": "CDKN1A"
}